{
  "gene": "UniProtKB:P31946",
  "gene_symbol": "YWHAB",
  "term_label": "signal transduction",
  "term_id": "GO:0007165",
  "gene_name": "14-3-3 protein beta_alpha"
}